{
  "term_label": "Unknown biological process",
  "gene_symbol": "GAGE6",
  "gene": "UniProtKB:Q13070",
  "term_id": "UNKNOWN:0002",
  "gene_name": "G antigen 6"
}